{
  "gene_name": "Transcription factor ATOH7",
  "gene_symbol": "ATOH7",
  "gene": "UniProtKB:Q8N100",
  "term_id": "GO:0005634",
  "term_label": "nucleus"
}